astrocyte end-foot [GO:0097450] (cellular component) Relationships: is a type of astrocyte projection [GO:0097449] Also known as: astrocyte endfoot Definition: Terminal process of astrocyte abutting non-neuronal surfaces in the brain. Subtypes: glial limiting end-foot [GO:0097451] Sources: NIF_Subcellular:sao388182739